{
  "term_label": "Unknown molecular function",
  "gene": "UniProtKB:A0A499FJF3",
  "gene_name": "Rho-GAP domain-containing protein",
  "gene_symbol": "A0A499FJF3",
  "term_id": "UNKNOWN:0001"
}